acetolactate synthase complex [GO:0005948] (cellular component) Definition: A dimeric (a large and a small chain) or tetrameric (two large and two small chains) enzyme complex. Catalyzes the formation of acetolactate from pyruvate. Relationships: is a type of transferase complex [GO:1990234]; is part of GO:0005737 References: PMID:16458324, PMID:8756689 Sources: GOC:jl Also known as: acetohydroxyacid synthase complex Note: See also the molecular function term 'acetolactate synthase activity ; GO:0003984'.